{
  "term_label": "Unknown biological process",
  "gene_name": "Asporin",
  "gene": "UniProtKB:Q9BXN1",
  "gene_symbol": "ASPN",
  "term_id": "UNKNOWN:0002"
}